{
  "term_label": "T cell receptor signaling pathway",
  "gene_name": "V-set domain-containing T-cell activation inhibitor 1",
  "gene": "UniProtKB:Q7Z7D3",
  "gene_symbol": "VTCN1",
  "term_id": "GO:0050852"
}